{
  "gene_symbol": "GJC1",
  "gene": "UniProtKB:P36383",
  "term_id": "GO:0005922",
  "gene_name": "Gap junction gamma-1 protein",
  "term_label": "connexin complex"
}